regulation of heart contraction involved in acute-phase response [GO:0002531] (biological process) Definition: Any process that modulates the frequency, rate or extent of heart contraction that contributes to the acute phase response. The acute phase response occurs during the early phases of an infection and is marked by changes in the production of plasma proteins such as C-reactive protein. References: PMID:15642986, PMID:15834430 Sources: GOC:jal Also known as: regulation of cardiac contraction during acute phase response, regulation of heart contraction during acute phase response Relationships: is a type of regulation of heart contraction [GO:0008016]; is part of acute-phase response [GO:0006953]